negative regulation of lymphocyte anergy [GO:0002912] (biological process) Also known as: down regulation of lymphocyte anergy, down-regulation of lymphocyte anergy, downregulation of lymphocyte anergy, inhibition of lymphocyte anergy Relationships: is_a negative regulation of tolerance induction [GO:0002644]; is a type of GO:0002911; RO_0002212 lymphocyte anergy [GO:0002249] Sources: GOC:add Definition: Any process that stops, prevents, or reduces the frequency, rate, or extent of lymphocyte anergy. Subtypes: negative regulation of T cell anergy [GO:0002668], GO:0002671